{
  "term_label": "triglyceride biosynthetic process",
  "gene": "UniProtKB:O75907",
  "term_id": "GO:0019432",
  "gene_name": "Diacylglycerol O-acyltransferase 1",
  "gene_symbol": "DGAT1"
}